{
  "term_id": "UNKNOWN:0002",
  "term_label": "Unknown biological process",
  "gene_name": "SCAN domain-containing protein 1",
  "gene_symbol": "SCAND1",
  "gene": "UniProtKB:P57086"
}